gamma-glutamyl-gamma-aminobutyrate hydrolase activity [GO:0033969] (molecular function) Relationships: is a type of hydrolase activity, acting on carbon-nitrogen (but not peptide) bonds, in linear amides [GO:0016811] Definition: Catalysis of the reaction: 4-(L-gamma-glutamylamino)butanoate + H2O = 4-aminobutanoate + L-glutamate. Sources: EC:3.5.1.94, RHEA:19737 Also known as: 4-(glutamylamino)butanoate amidohydrolase activity, PuuD, YcjL, gamma-glutamyl-GABA hydrolase activity